cellular response to ceramide [GO:0106097] (biological process) Definition: Any process that results in a change in state or activity of a cell (in terms of movement, secretion, enzyme production, gene expression, etc.) as a result of a ceramide stimulus. References: PMID:18006463 Relationships: is a type of GO:0071396